perisynaptic extracellular matrix [GO:0098966] (cellular component) Also known as: extrasynaptic extracellular matrix, perisynaptic ECM Definition: The portion of the extracellular matrix that lies within the perisynaptic space. Relationships: is a type of GO:0099535 Sources: GOC:dos Subtypes: GO:0072534